molting cycle [GO:0042303] (biological process) Sources: GOC:jl, ISBN:0198506732 Relationships: is a type of multicellular organismal process [GO:0032501] Subtypes: GO:0007591, molting cycle, collagen and cuticulin-based cuticle [GO:0018996], hair cycle [GO:0042633] Definition: The periodic casting off and regeneration of an outer covering of cuticle, feathers, hair, horns, skin, etc.